{
  "term_id": "GO:0004392",
  "gene_symbol": "HMOX1",
  "gene": "UniProtKB:P09601",
  "term_label": "heme oxygenase (decyclizing) activity",
  "gene_name": "Heme oxygenase 1"
}